{
  "gene_symbol": "SLA",
  "term_label": "signal transduction",
  "term_id": "GO:0007165",
  "gene": "UniProtKB:Q13239",
  "gene_name": "Src-like-adapter"
}